{
  "gene_name": "T cell receptor alpha variable 29_delta variable 5",
  "gene": "UniProtKB:P04437",
  "term_label": "peptide antigen binding",
  "gene_symbol": "TRAV29DV5",
  "term_id": "GO:0042605"
}